{
  "gene_name": "Protocadherin Fat 3",
  "term_id": "GO:0005912",
  "term_label": "adherens junction",
  "gene": "UniProtKB:Q8TDW7",
  "gene_symbol": "FAT3"
}